{
  "gene_name": "DDB1- and CUL4-associated factor 17",
  "gene_symbol": "DCAF17",
  "term_id": "UNKNOWN:0001",
  "term_label": "Unknown molecular function",
  "gene": "UniProtKB:Q5H9S7"
}